{
  "gene_symbol": "THOC2",
  "gene_name": "THO complex subunit 2",
  "term_id": "GO:0006406",
  "gene": "UniProtKB:Q8NI27",
  "term_label": "mRNA export from nucleus"
}